{
  "gene_symbol": "HOMER2",
  "gene_name": "Homer protein homolog 2",
  "term_label": "plasma membrane",
  "gene": "UniProtKB:Q9NSB8",
  "term_id": "GO:0005886"
}